2-oxo-4-hydroxy-4-carboxy-5-ureidoimidazoline decarboxylase activity [GO:0051997] (molecular function) Definition: Catalysis of the reaction: 5-hydroxy-2-oxo-4-ureido-2,5-dihydro-1H imidazole-5-carboxylate + H+ = S-allantoin + CO2. Relationships: is a type of carboxy-lyase activity [GO:0016831] Also known as: 4-(carbamoylamino)-5-hydroxy-2-oxo-2,5-dihydro-1H-imidazole-5-carboxylate decarboxylase activity, OHCU decarboxylase activity Sources: MetaCyc:RXN-6201